{
  "gene": "UniProtKB:Q9BQ16",
  "term_label": "regulation of cell-substrate adhesion",
  "term_id": "GO:0010810",
  "gene_symbol": "SPOCK3",
  "gene_name": "Testican-3"
}